regulation of osteoclast differentiation [GO:0045670] (biological process) Definition: Any process that modulates the frequency, rate or extent of osteoclast differentiation. Sources: GOC:go_curators Relationships: is_a regulation of myeloid leukocyte differentiation [GO:0002761]; RO_0002211 GO:0030316 Subtypes: negative regulation of osteoclast differentiation [GO:0045671], positive regulation of osteoclast differentiation [GO:0045672]